{
  "term_label": "immune response",
  "term_id": "GO:0006955",
  "gene_symbol": "MICA",
  "gene": "UniProtKB:Q29983",
  "gene_name": "MHC class I polypeptide-related sequence A"
}